{
  "term_id": "GO:0005886",
  "gene_symbol": "TRPM2",
  "term_label": "plasma membrane",
  "gene": "UniProtKB:O94759",
  "gene_name": "Transient receptor potential cation channel subfamily M member 2"
}